{
  "gene": "UniProtKB:Q9H5J0",
  "gene_name": "Zinc finger and BTB domain-containing protein 3",
  "term_id": "GO:0000981",
  "gene_symbol": "ZBTB3",
  "term_label": "DNA-binding transcription factor activity, RNA polymerase II-specific"
}